regulation of kidney smooth muscle cell differentiation [GO:2000356] (biological process) Definition: Any process that modulates the frequency, rate or extent of kidney smooth muscle cell differentiation. Subtypes: negative regulation of kidney smooth muscle cell differentiation [GO:2000357], positive regulation of kidney smooth muscle cell differentiation [GO:2000358] Sources: GOC:obol Relationships: is a type of regulation of smooth muscle cell differentiation [GO:0051150]; regulates kidney smooth muscle cell differentiation [GO:0072195]